{
  "term_label": "Unknown biological process",
  "term_id": "UNKNOWN:0002",
  "gene_name": "Arylamine N-acetyltransferase 1",
  "gene": "UniProtKB:P18440",
  "gene_symbol": "NAT1"
}